{
  "term_id": "GO:0098978",
  "gene_symbol": "DRD2",
  "term_label": "glutamatergic synapse",
  "gene_name": "D(2) dopamine receptor",
  "gene": "UniProtKB:P14416"
}